{
  "gene_symbol": "ZNF829",
  "gene": "UniProtKB:Q3KNS6",
  "term_id": "UNKNOWN:0003",
  "gene_name": "Zinc finger protein 829",
  "term_label": "Unknown cellular component"
}